histone H2AK15 ubiquitin ligase activity [GO:0140858] (molecular function) Note: Note that the residue position corresponds to the canonical human H2A2A histone (UniProtKB:Q6FI13); this residue is conserved across all eukaryotes. Residue 1 is the first residue following removal of the initiating Methionine (Met). Note that each histone is encoded by multiple genes, and sequences may vary across different genes within an organism. Also known as: histone ubiquitin ligase activity (H2A-K15 specific) Definition: Catalysis of the transfer of a ubiquitin molecule to histone 2A at the lysine-15 residue. Relationships: is a type of GO:0141053 References: PMID:22980979, PMID:28624371